cell wall pectin metabolic process [GO:0052546] (biological process) Relationships: is a type of pectin metabolic process [GO:0045488]; is part of plant-type cell wall organization [GO:0009664] Sources: GOC:ai Definition: The chemical reactions and pathways involving pectin, a polymer containing a backbone of alpha-1,4-linked D-galacturonic acid residues, as part of the organization and biogenesis of the cell wall. Also known as: cell wall pectin metabolism, cellulose and pectin-containing cell wall pectin metabolic process, pectin metabolism during cell wall biogenesis, plant-type cell wall pectin metabolic process Subtypes: rhamnogalacturonan I metabolic process [GO:0010395], GO:0052325 Regulation: regulated by regulation of cell wall pectin metabolic process [GO:1902066]